{
  "gene": "UniProtKB:Q6ZMZ0",
  "gene_symbol": "RNF19B",
  "term_id": "GO:0061630",
  "term_label": "ubiquitin protein ligase activity",
  "gene_name": "E3 ubiquitin-protein ligase RNF19B"
}